glucoside transmembrane transporter activity [GO:0042947] (molecular function) Sources: GOC:jl, GOC:mtg_transport, ISBN:0815340729 Relationships: is a type of GO:1901505; is part of glucoside transport [GO:0042946] Subtypes: alpha-glucoside transmembrane transporter activity [GO:0015151], beta-glucoside transmembrane transporter activity [GO:0015573], (+)-abscisic acid D-glucopyranosyl ester transmembrane transporter activity [GO:1902417] Definition: Enables the transfer of glucosides from one side of a membrane to the other. Glucosides are glycosides in which the sugar group is a glucose residue.